{
  "gene": "UniProtKB:Q6F5E8",
  "gene_name": "Capping protein, Arp2_3 and myosin-I linker protein 2",
  "gene_symbol": "CARMIL2",
  "term_id": "GO:0016477",
  "term_label": "cell migration"
}